{
  "gene": "UniProtKB:P38484",
  "term_label": "plasma membrane",
  "gene_name": "Interferon gamma receptor 2",
  "term_id": "GO:0005886",
  "gene_symbol": "IFNGR2"
}